{
  "gene_symbol": "ADAM9",
  "gene_name": "Disintegrin and metalloproteinase domain-containing protein 9",
  "term_id": "GO:0004222",
  "gene": "UniProtKB:Q13443",
  "term_label": "metalloendopeptidase activity"
}